{
  "gene_symbol": "DDR2",
  "gene_name": "Discoidin domain-containing receptor 2",
  "gene": "UniProtKB:Q16832",
  "term_id": "GO:0051897",
  "term_label": "positive regulation of phosphatidylinositol 3-kinase/protein kinase B signal transduction"
}